{
  "gene_symbol": "OR14C36",
  "gene": "UniProtKB:Q8NHC7",
  "term_label": "odorant binding",
  "term_id": "GO:0005549",
  "gene_name": "Olfactory receptor 14C36"
}